{
  "gene": "UniProtKB:P02776",
  "term_label": "antimicrobial humoral immune response mediated by antimicrobial peptide",
  "gene_symbol": "PF4",
  "gene_name": "Platelet factor 4",
  "term_id": "GO:0061844"
}